{
  "term_label": "Unknown molecular function",
  "gene": "UniProtKB:Q7Z553",
  "term_id": "UNKNOWN:0001",
  "gene_symbol": "MDGA2",
  "gene_name": "MAM domain-containing glycosylphosphatidylinositol anchor protein 2"
}